{
  "term_label": "cytosol",
  "gene_name": "Dual specificity protein phosphatase 15",
  "gene": "UniProtKB:Q9H1R2",
  "gene_symbol": "DUSP15",
  "term_id": "GO:0005829"
}